rolling circle single-stranded viral DNA replication [GO:0039684] (biological process) Sources: GOC:bf, GOC:jl, VZ:1941 Relationships: is_a rolling circle viral DNA replication [GO:0039682] Also known as: ssDNA rolling circle replication Definition: A rolling circle viral DNA replication that begins with a single-stranded viral DNA genome.